{
  "term_id": "GO:0005770",
  "gene_symbol": "SNX14",
  "gene_name": "Sorting nexin-14",
  "term_label": "late endosome",
  "gene": "UniProtKB:Q9Y5W7"
}